{
  "term_id": "GO:0005634",
  "term_label": "nucleus",
  "gene_name": "Steroid receptor-associated and regulated protein",
  "gene": "UniProtKB:Q8NEQ6",
  "gene_symbol": "SRARP"
}